{
  "term_id": "GO:0006357",
  "gene": "UniProtKB:P17040",
  "gene_symbol": "ZSCAN20",
  "gene_name": "Zinc finger and SCAN domain-containing protein 20",
  "term_label": "regulation of transcription by RNA polymerase II"
}